{
  "gene_symbol": "RGPD1",
  "gene_name": "RANBP2-like and GRIP domain-containing protein 1",
  "term_id": "GO:0006607",
  "gene": "UniProtKB:P0DJD0",
  "term_label": "NLS-bearing protein import into nucleus"
}